{
  "term_id": "GO:0017154",
  "term_label": "semaphorin receptor activity",
  "gene": "UniProtKB:P51805",
  "gene_name": "Plexin-A3",
  "gene_symbol": "PLXNA3"
}